histone H2BK12 acetyltransferase activity [GO:0044015] (molecular function) Note: Note that the residue position corresponds to the canonical human H2B histone (UniProtKB:P62807); the N-terminus of histone H2B is divergent across eukaryotes; make sure that the paper clearly references the human protein for the position of this modification to use this term. Residue 1 is the first residue following removal of the initiating Methionine (Met). Note that each histone is encoded by multiple genes, and sequences may vary across different genes within an organism. Also known as: histone H2B-K12 acetyltransferase activity, histone acetylase activity (H2B-K12 specific), histone acetyltransferase activity (H2B-K12 specific), histone lysine N-acetyltransferase activity (H2B-K12 specific) References: PMID:18552846 Relationships: is a type of histone H2B acetyltransferase activity [GO:0044013] Definition: Catalysis of the reaction: acetyl-CoA + histone H2B L-lysine (position 12) = CoA + histone H2B N6-acetyl-L-lysine (position 12).